{
  "term_id": "GO:0007420",
  "gene_name": "Pre-B-cell leukemia transcription factor 3",
  "gene": "UniProtKB:P40426",
  "term_label": "brain development",
  "gene_symbol": "PBX3"
}